{
  "term_label": "leptin-mediated signaling pathway",
  "gene": "UniProtKB:P40763",
  "term_id": "GO:0033210",
  "gene_name": "Signal transducer and activator of transcription 3",
  "gene_symbol": "STAT3"
}